cellular detoxification of fluoride [GO:0140114] (biological process) Relationships: is a type of detoxification of inorganic compound [GO:0061687]; is a type of cellular detoxification [GO:1990748]; is part of GO:1902618 Definition: Any process carried out at the cellular level that reduces or removes the toxicity of a fluoride. These may include chemical modification or transport of fluoride away from sensitive areas and to compartments or complexes whose purpose is sequestration of the toxic substance. Sources: GOC:vw